{
  "gene_symbol": "TMEM253",
  "term_id": "UNKNOWN:0002",
  "gene_name": "Transmembrane protein 253",
  "gene": "UniProtKB:P0C7T8",
  "term_label": "Unknown biological process"
}